{
  "gene_symbol": "CASKIN2",
  "term_label": "Unknown cellular component",
  "gene": "UniProtKB:Q8WXE0",
  "term_id": "UNKNOWN:0003",
  "gene_name": "Caskin-2"
}